{
  "term_label": "negative regulation of gene expression",
  "gene_symbol": "CCDC3",
  "term_id": "GO:0010629",
  "gene": "UniProtKB:Q9BQI4",
  "gene_name": "Coiled-coil domain-containing protein 3"
}